{
  "term_id": "GO:0000981",
  "gene_symbol": "SIM2",
  "gene_name": "Single-minded homolog 2",
  "term_label": "DNA-binding transcription factor activity, RNA polymerase II-specific",
  "gene": "UniProtKB:Q14190"
}